{
  "gene_symbol": "EIF1AY",
  "term_label": "translational initiation",
  "gene": "UniProtKB:O14602",
  "term_id": "GO:0006413",
  "gene_name": "Eukaryotic translation initiation factor 1A, Y-chromosomal"
}